{
  "gene_name": "Fibroblast growth factor 8",
  "gene": "UniProtKB:P55075",
  "term_id": "GO:0005615",
  "gene_symbol": "FGF8",
  "term_label": "extracellular space"
}